capsule polysaccharide biosynthetic process [GO:0045227] (BP) Relationships: is a type of polysaccharide biosynthetic process [GO:0000271]; is a type of capsule organization [GO:0045230] Sources: GOC:go_curators Regulation: regulated by regulation of capsule polysaccharide biosynthetic process [GO:0062084]; positively regulated by positive regulation of capsule polysaccharide biosynthetic process [GO:0062085] Definition: The chemical reactions and pathways resulting in the formation of polysaccharides that make up the capsule, a protective structure surrounding some species of bacteria and fungi. Also known as: capsular polysaccharide biosynthesis, capsular polysaccharide biosynthetic process, capsule polysaccharide anabolism, capsule polysaccharide biosynthesis, capsule polysaccharide formation, capsule polysaccharide synthesis